{
  "gene_name": "ATP-dependent DNA_RNA helicase DHX36",
  "term_id": "GO:0051880",
  "gene_symbol": "DHX36",
  "gene": "UniProtKB:Q9H2U1",
  "term_label": "G-quadruplex DNA binding"
}